{
  "gene": "UniProtKB:Q9BRK3",
  "term_label": "cell surface",
  "gene_name": "Matrix remodeling-associated protein 8",
  "gene_symbol": "MXRA8",
  "term_id": "GO:0009986"
}